viral procapsid maturation [GO:0046797] (biological process) Also known as: virion maturation, capsid maturation, viral capsid maturation References: PMID:10627558, PMID:19204733 Sources: GOC:bf Relationships: is a type of cellular component assembly [GO:0022607]; is part of viral capsid assembly [GO:0019069]; is part of GO:0019075 Definition: The refolding and structural rearrangements of individual capsid subunits to transition from the intermediate procapsid, to the more stable capsid structure.